{
  "term_label": "receptor ligand activity",
  "gene_name": "UL-16 binding protein 5",
  "gene_symbol": "RAET1G",
  "gene": "UniProtKB:Q6H3X3",
  "term_id": "GO:0048018"
}